response to 4-nitroquinoline N-oxide [GO:0072724] (biological process) Definition: Any process that results in a change in state or activity of a cell or an organism (in terms of movement, secretion, enzyme production, gene expression, etc.) as a result of a 4-nitroquinoline N-oxide stimulus. Sources: GOC:mah Relationships: is a type of response to nitrogen compound [GO:1901698]; is a type of response to oxygen-containing compound [GO:1901700] Subtypes: GO:0072725